{
  "term_label": "glycogen metabolic process",
  "gene_name": "UTP--glucose-1-phosphate uridylyltransferase",
  "gene": "UniProtKB:Q16851",
  "gene_symbol": "UGP2",
  "term_id": "GO:0005977"
}